{
  "term_label": "plasma membrane",
  "term_id": "GO:0005886",
  "gene_symbol": "JPH4",
  "gene_name": "Junctophilin-4",
  "gene": "UniProtKB:Q96JJ6"
}